Bolwig's organ development [GO:0055034] (biological process) Definition: The process whose specific outcome is the progression of the Bolwig's organ over time, from its formation to the mature structure. The larval eye in Drosophila is a relatively simple sensory system composed of Bolwig's organs: two clusters, each composed of 12 photoreceptor cells from which axons extend in a single fascicle to the brain. Relationships: is a type of eye development [GO:0001654] Sources: GOC:mtg_sensu